telomerase catalytic core complex [GO:0000333] (cellular component) Also known as: TERT-TERC complex Definition: The minimal catalytic core of telomerase is a ribonucleoprotein complex composed of a catalytic reverse transcriptase subunit and an RNA subunit that provides the template for telomeric DNA addition. References: PMID:11884619, PMID:1808260 Sources: GOC:BHF-UCL Relationships: is a type of GO:0005697; is a type of GO:0061695